short-chain fatty acyl-CoA dehydrogenase activity [GO:0016937] (molecular function) Note: While there is not universal consensus on the lengths of short-, medium-, long- and very-long-chain fatty acids, the GO uses the definitions in ChEBI (see CHEBI:26666, CHEBI:59554, CHEBI:15904 and CHEBI:27283). Subtypes: short-chain 2-methyl fatty acyl-CoA dehydrogenase activity [GO:0003853], 3-methylbutanoyl-CoA dehydrogenase activity [GO:0008470] Definition: Catalysis of the reaction: a short-chain 2,3-saturated fatty acyl-CoA + H+ + oxidized [electron-transfer flavoprotein] = a short-chain (2E)-enoyl-CoA + reduced [electron-transfer flavoprotein]. A short-chain fatty acid has an aliphatic tail containing fewer than 6 carbons. Relationships: is a type of acyl-CoA dehydrogenase activity [GO:0003995] Also known as: unsaturated acyl-CoA reductase, short-chain acyl CoA dehydrogenase, short-chain-acyl-CoA dehydrogenase activity, butanoyl-CoA dehydrogenase, butyryl dehydrogenase Sources: RHEA:47196